{
  "term_label": "Swr1 complex",
  "gene_symbol": "ZNHIT1",
  "gene_name": "Zinc finger HIT domain-containing protein 1",
  "term_id": "GO:0000812",
  "gene": "UniProtKB:O43257"
}